{
  "term_label": "hair cycle",
  "term_id": "GO:0042633",
  "gene": "UniProtKB:G5E9R7",
  "gene_name": "Putative keratin-associated protein 4-16",
  "gene_symbol": "KRTAP4-16"
}